{
  "term_label": "uridine phosphorylase activity",
  "gene_symbol": "UPP2",
  "gene": "UniProtKB:O95045",
  "term_id": "GO:0004850",
  "gene_name": "Uridine phosphorylase 2"
}